{
  "term_id": "GO:0007608",
  "gene": "UniProtKB:Q8NGG3",
  "gene_name": "Olfactory receptor 5T3",
  "term_label": "sensory perception of smell",
  "gene_symbol": "OR5T3"
}